positive regulation of mitotic cell cycle, embryonic [GO:0045977] (biological process) Sources: GOC:dph, GOC:go_curators, GOC:tb Subtypes: positive regulation of preblastoderm mitotic cell cycle [GO:0046002], positive regulation of syncytial blastoderm mitotic cell cycle [GO:0046004] Also known as: positive regulation of embryonic mitotic cell cycle, positive regulation of embryonic mitotic cell cycle progression, positive regulation of progression through embryonic mitotic cell cycle, up regulation of mitotic cell cycle, embryonic, up-regulation of mitotic cell cycle, embryonic, upregulation of mitotic cell cycle, embryonic, activation of mitotic cell cycle, embryonic, stimulation of mitotic cell cycle, embryonic Definition: Any process that activates or increases the frequency, rate or extent of progression through the embryonic mitotic cell cycle. Relationships: is a type of GO:0009794; is a type of positive regulation of mitotic cell cycle [GO:0045931]; positively regulates mitotic cell cycle, embryonic [GO:0045448]